G protein-coupled serotonin receptor binding [GO:0031821] (molecular function) Relationships: is a type of G protein-coupled receptor binding [GO:0001664] Also known as: G-protein coupled serotonin receptor binding, metabotropic 5-hydroxytryptamine receptor binding, metabotropic serotonin receptor binding, metabotropic serotonin receptor ligand Definition: Binding to a metabotropic serotonin receptor. Subtypes: GO:0031822, type 1D serotonin receptor binding [GO:0031823], type 1E serotonin receptor binding [GO:0031824], type 1F serotonin receptor binding [GO:0031825], type 2A serotonin receptor binding [GO:0031826], type 2B serotonin receptor binding [GO:0031827], type 2C serotonin receptor binding [GO:0031828], GO:0031829, type 5A serotonin receptor binding [GO:0031830], type 5B serotonin receptor binding [GO:0031831], GO:0031832, type 7 serotonin receptor binding [GO:0031833] Sources: GOC:mah, GOC:nln